{
  "gene_symbol": "NCK2",
  "gene": "UniProtKB:O43639",
  "term_id": "GO:0036493",
  "gene_name": "Cytoplasmic protein NCK2",
  "term_label": "positive regulation of translation in response to endoplasmic reticulum stress"
}